{
  "term_id": "GO:0000978",
  "gene_name": "Zinc finger protein 549",
  "gene_symbol": "ZNF549",
  "term_label": "RNA polymerase II cis-regulatory region sequence-specific DNA binding",
  "gene": "UniProtKB:Q6P9A3"
}